{
  "gene_name": "Ras-related C3 botulinum toxin substrate 3",
  "gene_symbol": "RAC3",
  "term_id": "GO:0043005",
  "gene": "UniProtKB:P60763",
  "term_label": "neuron projection"
}